{
  "gene": "UniProtKB:P56915",
  "term_id": "GO:0005634",
  "term_label": "nucleus",
  "gene_symbol": "GSC",
  "gene_name": "Homeobox protein goosecoid"
}